{
  "gene_symbol": "IL2RB",
  "term_id": "GO:0004911",
  "gene_name": "Interleukin-2 receptor subunit beta",
  "term_label": "interleukin-2 receptor activity",
  "gene": "UniProtKB:P14784"
}